{
  "gene": "UniProtKB:O75438",
  "term_id": "GO:0045271",
  "term_label": "respiratory chain complex I",
  "gene_name": "NADH dehydrogenase [ubiquinone] 1 beta subcomplex subunit 1",
  "gene_symbol": "NDUFB1"
}